{
  "term_id": "GO:0005886",
  "gene": "UniProtKB:Q9ULV8",
  "gene_name": "E3 ubiquitin-protein ligase CBL-C",
  "term_label": "plasma membrane",
  "gene_symbol": "CBLC"
}